{
  "gene": "UniProtKB:Q9UKU7",
  "term_id": "UNKNOWN:0003",
  "term_label": "Unknown cellular component",
  "gene_symbol": "ACAD8",
  "gene_name": "Isobutyryl-CoA dehydrogenase, mitochondrial"
}